{
  "gene_symbol": "STRIT1",
  "gene_name": "Sarcoplasmic_endoplasmic reticulum calcium ATPase regulator DWORF",
  "term_id": "UNKNOWN:0003",
  "term_label": "Unknown cellular component",
  "gene": "UniProtKB:P0DN84"
}